C1 axonemal microtubule [GO:1990719] (cellular component) Relationships: is a type of axonemal microtubule [GO:0005879]; is part of axonemal central pair [GO:0097540] References: PMID:21586547, PMID:9295136 Sources: GOC:cilia Definition: One of two microtubules present in the axonemal central pair. It is distinguishable from the C2 axonemal microtubule (also called C2 tubule) by the presence of differing protein components of the projections. Also known as: C1 tubule